{
  "term_label": "egg coat",
  "gene_symbol": "ZP2",
  "gene": "UniProtKB:Q05996",
  "term_id": "GO:0035805",
  "gene_name": "Zona pellucida sperm-binding protein 2"
}